{
  "term_label": "Unknown cellular component",
  "gene_name": "Nucleus accumbens-associated protein 1",
  "term_id": "UNKNOWN:0003",
  "gene_symbol": "NACC1",
  "gene": "UniProtKB:Q96RE7"
}